phospho-N-acetylmuramoyl-pentapeptide-transferase activity [GO:0008963] (molecular function) Also known as: MraY transferase activity, UDP-MurAc(oyl-L-Ala-gamma-D-Glu-L-Lys-D-Ala-D-Ala):undecaprenyl-phosphate phospho-N-acetylmuramoyl-pentapeptide-transferase activity, UDP-MurNAc-Ala-gamma-DGlu-Lys-DAla-DAla:undecaprenylphosphate transferase activity, UDP-MurNAc-Ala-gammaDGlu-Lys-DAla-DAla:undecaprenylphosphate transferase activity, UDP-MurNAc-L-Ala-D-gamma-Glu-L-Lys-D-Ala-D-Ala:C(55)-isoprenoid alcohol transferase activity, UDP-MurNAc-L-Ala-D-gamma-Glu-L-Lys-D-Ala-D-Ala:C55-isoprenoid alcohol transferase activity, UDP-MurNAc-pentapeptide phosphotransferase activity, phospho-MurNAc-pentapeptide transferase activity, phospho-N-acetylmuramoyl pentapeptide translocase activity, phospho-NAc-muramoyl-pentapeptide translocase (UMP) activity, phosphoacetylmuramoylpentapeptide translocase activity, phosphoacetylmuramoylpentapeptidetransferase activity Definition: Catalysis of the reaction: di-trans,octa-cis-undecaprenyl phosphate + UDP-N-acetyl-alpha-D-muramoyl-L-alanyl-gamma-D-glutamyl-L-lysyl-D-alanyl-D-alanine = Mur2Ac(oyl-L-Ala-gamma-D-Glu-L-Lys-D-Ala-D-Ala)-di-trans,octa-cis-undecaprenyl diphosphate + UMP. Relationships: is a type of phosphotransferase activity, for other substituted phosphate groups [GO:0016780] Sources: RHEA:21920 Note: Note that EC classifies all three 'UDP-N-acetylmuramoyl-L-alanyl-D-glutamyl-meso-2,6-diaminopimelyl-D-alanyl-D-alanine:undecaprenyl-phosphate transferase activity ; GO:0051992' and 'phospho-N-acetylmuramoyl-pentapeptide-transferase activity ; GO:0008963' under EC:2.7.8.13.